triacetate-lactonase activity [GO:0050349] (molecular function) Relationships: is a type of carboxylic ester hydrolase activity [GO:0052689] Also known as: TAL hydrolase activity, triacetate lactone hydrolase activity, triacetic acid lactone hydrolase activity, triacetic lactone hydrolase activity, triacetolactone lactonohydrolase activity Definition: Catalysis of the reaction: H2O + triacetate lactone = triacetate. Sources: EC:3.1.1.38, RHEA:22260